{
  "gene_symbol": "OR2B6",
  "gene": "UniProtKB:P58173",
  "term_label": "plasma membrane",
  "term_id": "GO:0005886",
  "gene_name": "Olfactory receptor 2B6"
}